{
  "term_label": "intraciliary retrograde transport",
  "gene_symbol": "DYNLL1",
  "gene_name": "Dynein light chain 1, cytoplasmic",
  "gene": "UniProtKB:P63167",
  "term_id": "GO:0035721"
}